{
  "gene": "UniProtKB:P23759",
  "gene_symbol": "PAX7",
  "gene_name": "Paired box protein Pax-7",
  "term_id": "UNKNOWN:0003",
  "term_label": "Unknown cellular component"
}